{
  "gene_name": "EGF-containing fibulin-like extracellular matrix protein 1",
  "gene_symbol": "EFEMP1",
  "term_label": "extracellular matrix",
  "term_id": "GO:0031012",
  "gene": "UniProtKB:Q12805"
}